positive regulation of Atg1/ULK1 kinase complex assembly [GO:1905866] (biological process) Also known as: positive regulation of ATG1 kinase complex assembly, positive regulation of ATG1 kinase complex formation, positive regulation of ATG1-ATG13 complex assembly, positive regulation of ATG1-ATG13 complex formation, positive regulation of ATG1/ULK1 kinase complex formation, positive regulation of ATG1/ULK1 signaling complex assembly, positive regulation of ATG1/ULK1 signaling complex formation, positive regulation of Atg1p signalling complex assembly, positive regulation of Atg1p signalling complex formation, positive regulation of ULK1 signaling complex assembly, positive regulation of ULK1 signaling complex formation, positive regulation of ULK1-ATG13-FIP200 complex assembly, positive regulation of ULK1-ATG13-FIP200 complex formation, positive regulation of ULK1-ATG13-RB1CC1 complex assembly, positive regulation of ULK1-ATG13-RB1CC1 complex formation, up regulation of ATG1 kinase complex assembly, up regulation of ATG1 kinase complex formation, up regulation of ATG1-ATG13 complex assembly, up regulation of ATG1-ATG13 complex formation, up regulation of ATG1/ULK1 kinase complex assembly, up regulation of ATG1/ULK1 kinase complex formation, up regulation of ATG1/ULK1 signaling complex assembly, up regulation of ATG1/ULK1 signaling complex formation, up regulation of Atg1p signalling complex assembly, up regulation of Atg1p signalling complex formation, up regulation of ULK1 signaling complex assembly, up regulation of ULK1 signaling complex formation, up regulation of ULK1-ATG13-FIP200 complex assembly, up regulation of ULK1-ATG13-FIP200 complex formation, up regulation of ULK1-ATG13-RB1CC1 complex assembly, up regulation of ULK1-ATG13-RB1CC1 complex formation, up-regulation of ATG1 kinase complex assembly, up-regulation of ATG1 kinase complex formation, up-regulation of ATG1-ATG13 complex assembly, up-regulation of ATG1-ATG13 complex formation, up-regulation of ATG1/ULK1 kinase complex assembly, up-regulation of ATG1/ULK1 kinase complex formation, up-regulation of ATG1/ULK1 signaling complex assembly, up-regulation of ATG1/ULK1 signaling complex formation, up-regulation of Atg1p signalling complex assembly, up-regulation of Atg1p signalling complex formation, up-regulation of ULK1 signaling complex assembly, up-regulation of ULK1 signaling complex formation, up-regulation of ULK1-ATG13-FIP200 complex assembly, up-regulation of ULK1-ATG13-FIP200 complex formation, up-regulation of ULK1-ATG13-RB1CC1 complex assembly, up-regulation of ULK1-ATG13-RB1CC1 complex formation, upregulation of ATG1 kinase complex assembly, upregulation of ATG1 kinase complex formation, upregulation of ATG1-ATG13 complex assembly, upregulation of ATG1-ATG13 complex formation, upregulation of ATG1/ULK1 kinase complex assembly, upregulation of ATG1/ULK1 kinase complex formation, upregulation of ATG1/ULK1 signaling complex assembly, upregulation of ATG1/ULK1 signaling complex formation, upregulation of Atg1p signalling complex assembly, upregulation of Atg1p signalling complex formation, upregulation of ULK1 signaling complex assembly, upregulation of ULK1 signaling complex formation, upregulation of ULK1-ATG13-FIP200 complex assembly, upregulation of ULK1-ATG13-FIP200 complex formation, upregulation of ULK1-ATG13-RB1CC1 complex assembly, upregulation of ULK1-ATG13-RB1CC1 complex formation, activation of ATG1 kinase complex assembly, activation of ATG1 kinase complex formation, activation of ATG1-ATG13 complex assembly, activation of ATG1-ATG13 complex formation, activation of ATG1/ULK1 kinase complex assembly, activation of ATG1/ULK1 kinase complex formation, activation of ATG1/ULK1 signaling complex assembly, activation of ATG1/ULK1 signaling complex formation, activation of Atg1p signalling complex assembly, activation of Atg1p signalling complex formation, activation of ULK1 signaling complex assembly, activation of ULK1 signaling complex formation, activation of ULK1-ATG13-FIP200 complex assembly, activation of ULK1-ATG13-FIP200 complex formation, activation of ULK1-ATG13-RB1CC1 complex assembly, activation of ULK1-ATG13-RB1CC1 complex formation Relationships: is a type of positive regulation of protein-containing complex assembly [GO:0031334]; is a type of regulation of Atg1/ULK1 kinase complex assembly [GO:1905864]; positively regulates Atg1/ULK1 kinase complex assembly [GO:1904745] References: PMID:26567215 Sources: GOC:TermGenie, GOC:autophagy, GOC:mf, GO_REF:0000058 Definition: Any process that activates or increases the frequency, rate or extent of Atg1/ULK1 kinase complex assembly.